{
  "gene": "UniProtKB:Q8NDX5",
  "term_id": "GO:0035102",
  "gene_symbol": "PHC3",
  "term_label": "PRC1 complex",
  "gene_name": "Polyhomeotic-like protein 3"
}